oxidoreductase activity, acting on diphenols and related substances as donors [GO:0016679] (molecular function) Relationships: is_a GO:0016491 Also known as: oxidoreductase activity, acting on diphenols and related substances as donors, other acceptors Sources: GOC:ai Subtypes: dihydronicotinamide riboside quinone reductase activity [GO:0001512], GO:0016680, GO:0016682, oxidoreductase activity, acting on diphenols and related substances as donors, with copper protein as acceptor [GO:0052880] Definition: Catalysis of an oxidation-reduction (redox) reaction in which a diphenol or related substance acts as a hydrogen or electron donor and reduces a hydrogen or electron acceptor.